degradation of host chromosome by virus [GO:0099015] (biological process) Relationships: is a type of viral process [GO:0016032]; is part of GO:0039693 References: PMID:163355, PMID:335083, PMID:3972821, PMID:5263754 Sources: VZ:3947 Definition: The catabolic breakdown of the DNA of a host chromosome by a virus. This occurs during infection of bacteria by some phages. It frees up a large pool of nucleoside 5'-triphophates for use in viral DNA synthesis.